{
  "gene": "UniProtKB:Q13976",
  "gene_name": "cGMP-dependent protein kinase 1",
  "term_label": "signal transduction",
  "gene_symbol": "PRKG1",
  "term_id": "GO:0007165"
}